{
  "term_label": "protein localization to cilium",
  "term_id": "GO:0061512",
  "gene_name": "Tetratricopeptide repeat protein 21B",
  "gene_symbol": "TTC21B",
  "gene": "UniProtKB:Q7Z4L5"
}